mitochondrial mRNA modification [GO:0080156] (biological process) References: PMID:20566637 Definition: The covalent alteration within the mitochondrion of one or more nucleotides within an mRNA to produce an mRNA molecule with a sequence that differs from that coded genetically. Also known as: mitochondrial RNA editing, mitochondrial mRNA editing Relationships: is a type of mRNA modification [GO:0016556]; is a type of GO:1900864